negative regulation of negative chemotaxis [GO:0050925] (biological process) Sources: GOC:ai Relationships: is a type of negative regulation of chemotaxis [GO:0050922]; is a type of regulation of negative chemotaxis [GO:0050923]; negatively regulates negative chemotaxis [GO:0050919] Also known as: down regulation of negative chemotaxis, down-regulation of negative chemotaxis, downregulation of negative chemotaxis, inhibition of negative chemotaxis Definition: Any process that stops, prevents, or reduces the frequency, rate or extent of the directed movement of a motile cell or organism towards a lower concentration in a concentration gradient of a specific chemical.